{
  "gene_name": "Ras-related protein Rab-3A",
  "term_label": "axon",
  "gene": "UniProtKB:P20336",
  "gene_symbol": "RAB3A",
  "term_id": "GO:0030424"
}